{
  "gene_name": "Coiled-coil domain-containing protein 127",
  "term_id": "UNKNOWN:0001",
  "gene": "UniProtKB:Q96BQ5",
  "term_label": "Unknown molecular function",
  "gene_symbol": "CCDC127"
}